pyridoxamine binding [GO:0070281] (molecular function) Sources: CHEBI:16410, GOC:mah Relationships: is a type of cation binding [GO:0043169]; is a type of vitamin B6 binding [GO:0070279] Definition: Binding to pyridoxamine, 4-(aminomethyl)-5-(hydroxymethyl)-2-methylpyridin-3-ol, a form of vitamin B6.